{
  "gene_name": "Melanin-concentrating hormone receptor 1",
  "gene_symbol": "MCHR1",
  "gene": "UniProtKB:Q99705",
  "term_label": "G protein-coupled receptor activity",
  "term_id": "GO:0004930"
}